somatodendritic compartment [GO:0036477] (cellular component) Sources: GOC:PARL, GOC:pad Definition: The region of a neuron that includes the cell body (cell soma) and dendrite(s), but excludes the axon. Relationships: is a type of GO:0110165